{
  "term_id": "GO:0007605",
  "gene_name": "Calcium-binding protein 4",
  "gene_symbol": "CABP4",
  "term_label": "sensory perception of sound",
  "gene": "UniProtKB:P57796"
}